myosin I complex [GO:0045160] (cellular component) References: PMID:9438839 Sources: GOC:mah Definition: A myosin complex containing a class I myosin heavy chain and associated light chains; myosin I heavy chains are single-headed, possess tails of various lengths, and do not self-associate into bipolar filaments; myosin I complexes are involved in diverse processes related to membrane traffic and cell movement. Relationships: is a type of unconventional myosin complex [GO:0016461]